N-glycan processing [GO:0006491] (biological process) Also known as: N-linked glycoprotein maturation, glycoprotein trimming involved in glycoprotein maturation Definition: The conversion of N-linked glycan (N = nitrogen) structures from the initially transferred oligosaccharide to a mature form, by the actions of glycosidases and glycosyltransferases. The early processing steps are conserved and play roles in glycoprotein folding and trafficking. References: PMID:12736198, PMID:35536965 Subtypes: N-glycan processing to lysosome [GO:0016256], Golgi apparatus N-glycan diversification [GO:0016258], GO:0140277, Golgi apparatus N-glycan mannose trimming [GO:1904381] Relationships: is a type of glycoprotein biosynthetic process [GO:0009101]; is part of protein N-linked glycosylation [GO:0006487]